positive regulation of interleukin-23 production [GO:0032747] (biological process) Sources: GOC:mah Relationships: is a type of GO:0001819; is a type of regulation of interleukin-23 production [GO:0032667]; RO_0002213 interleukin-23 production [GO:0032627] Also known as: positive regulation of IL-23 production, up regulation of interleukin-23 production, up-regulation of interleukin-23 production, upregulation of interleukin-23 production, activation of interleukin-23 production, positive regulation of interleukin-23 biosynthetic process, stimulation of interleukin-23 production Definition: Any process that activates or increases the frequency, rate, or extent of interleukin-23 production.